{
  "term_label": "immune response",
  "gene": "UniProtKB:P0DSN7",
  "term_id": "GO:0006955",
  "gene_name": "Probable non-functional immunoglobulinn kappa variable 1D-37",
  "gene_symbol": "IGKV1D-37"
}